positive regulation of amylopectin catabolic process [GO:2000947] (biological process) Also known as: positive regulation of Amylopectin catabolism Sources: GOC:mengo_curators Definition: Any process that activates or increases the frequency, rate or extent of amylopectin catabolic process. Relationships: is a type of positive regulation of starch catabolic process [GO:2000883]; is a type of regulation of amylopectin catabolic process [GO:2000945]; positively regulates amylopectin catabolic process [GO:2000897]